{
  "term_label": "positive regulation of mitotic nuclear division",
  "gene_symbol": "BTC",
  "gene_name": "Probetacellulin",
  "term_id": "GO:0045840",
  "gene": "UniProtKB:P35070"
}